{
  "term_label": "protein serine/threonine kinase activity",
  "gene_name": "Serine_threonine-protein kinase RIO1",
  "term_id": "GO:0004674",
  "gene_symbol": "RIOK1",
  "gene": "UniProtKB:Q9BRS2"
}